{
  "gene": "UniProtKB:Q96R67",
  "term_label": "olfactory receptor activity",
  "gene_symbol": "OR4C12",
  "gene_name": "Olfactory receptor 4C12",
  "term_id": "GO:0004984"
}